{
  "gene": "UniProtKB:Q8IYB7",
  "gene_name": "DIS3-like exonuclease 2",
  "gene_symbol": "DIS3L2",
  "term_id": "GO:0000175",
  "term_label": "3'-5'-RNA exonuclease activity"
}